cytosolic region [GO:0099522] (cellular component) Sources: GOC:dos Subtypes: GO:0099523, postsynaptic cytosol [GO:0099524] Relationships: is a type of cytosol [GO:0005829]; is part of cytosol [GO:0005829] Definition: Any (proper) part of the cytosol of a single cell of sufficient size to still be considered cytosol. Also known as: region of cytosol